{
  "gene": "UniProtKB:P52952",
  "term_id": "GO:0000981",
  "term_label": "DNA-binding transcription factor activity, RNA polymerase II-specific",
  "gene_symbol": "NKX2-5",
  "gene_name": "Homeobox protein Nkx-2.5"
}